{
  "gene_name": "Carboxypeptidase A4",
  "term_label": "metallocarboxypeptidase activity",
  "gene_symbol": "CPA4",
  "gene": "UniProtKB:Q9UI42",
  "term_id": "GO:0004181"
}